{
  "term_id": "GO:1902983",
  "term_label": "DNA strand elongation involved in mitotic DNA replication",
  "gene_symbol": "GINS1",
  "gene": "UniProtKB:Q14691",
  "gene_name": "DNA replication complex GINS protein PSF1"
}